transmembrane transporter binding [GO:0044325] (molecular function) Relationships: is a type of GO:0005515 Definition: Binding to a transmembrane transporter, a protein or protein complex that enables the transfer of a substance, usually a specific substance or a group of related substances, from one side of a membrane to the other. Also known as: ion channel binding References: PMID:33199372 Sources: GOC:BHF, GOC:jl